{
  "term_label": "myelination",
  "gene_symbol": "CMTM8",
  "term_id": "GO:0042552",
  "gene_name": "CKLF-like MARVEL transmembrane domain-containing protein 8",
  "gene": "UniProtKB:Q8IZV2"
}